negative regulation of hepatocyte growth factor receptor signaling pathway [GO:1902203] (biological process) Also known as: down regulation of HGF receptor signaling pathway, down regulation of HGF receptor signalling pathway, down regulation of hepatocyte growth factor receptor signaling pathway, down-regulation of HGF receptor signaling pathway, down-regulation of HGF receptor signalling pathway, down-regulation of hepatocyte growth factor receptor signaling pathway, downregulation of HGF receptor signaling pathway, downregulation of HGF receptor signalling pathway, downregulation of hepatocyte growth factor receptor signaling pathway, inhibition of HGF receptor signaling pathway, inhibition of HGF receptor signalling pathway, negative regulation of HGF receptor signaling pathway, negative regulation of HGF receptor signalling pathway, down regulation of Met signaling pathway, down-regulation of Met signaling pathway, downregulation of Met signaling pathway, inhibition of Met signaling pathway, inhibition of hepatocyte growth factor receptor signaling pathway, negative regulation of Met signaling pathway Definition: Any process that stops, prevents or reduces the frequency, rate or extent of hepatocyte growth factor receptor signaling pathway. Relationships: is_a negative regulation of signal transduction [GO:0009968]; is a type of regulation of hepatocyte growth factor receptor signaling pathway [GO:1902202]; negatively regulates hepatocyte growth factor receptor signaling pathway [GO:0048012] References: PMID:18819921 Sources: GOC:TermGenie